C5-methylcytidine-containing RNA reader activity [GO:0062153] (molecular function) Relationships: is a type of GO:0140517; has part RNA binding [GO:0003723] References: PMID:28418038 Definition: A protein adaptor that recognizes and binds an RNA molecule modified by C5-methylcytidine. Also known as: C5-methylcytidine-containing RNA binding, C5-methylcytosine-containing RNA binding